endochondral bone morphogenesis [GO:0060350] (biological process) Definition: The process in which bones are generated and organized as a result of the conversion of initial cartilaginous anlage into bone. References: PMID:11680679 Sources: GOC:dph Relationships: is a type of bone morphogenesis [GO:0060349]